regulation of mesenchymal cell apoptotic process [GO:2001053] (biological process) Sources: GOC:mtg_apoptosis, GOC:obol Definition: Any process that modulates the frequency, rate or extent of mesenchymal cell apoptotic process. Subtypes: regulation of mesenchymal cell apoptotic process involved in nephron morphogenesis [GO:0072039], regulation of mesenchymal cell apoptotic process involved in metanephros development [GO:1900211], negative regulation of mesenchymal cell apoptotic process [GO:2001054], positive regulation of mesenchymal cell apoptotic process [GO:2001055] Also known as: regulation of mesenchymal cell apoptosis Relationships: is a type of regulation of apoptotic process [GO:0042981]; regulates GO:0097152